{
  "gene": "UniProtKB:Q9HCH5",
  "gene_symbol": "SYTL2",
  "term_label": "exocytic vesicle",
  "gene_name": "Synaptotagmin-like protein 2",
  "term_id": "GO:0070382"
}